{
  "gene": "UniProtKB:A0A0B4J235",
  "gene_name": "T cell receptor alpha variable 13-2",
  "term_id": "GO:0009617",
  "gene_symbol": "TRAV13-2",
  "term_label": "response to bacterium"
}